{
  "term_id": "GO:0036064",
  "gene": "UniProtKB:Q15154",
  "gene_name": "Pericentriolar material 1 protein",
  "gene_symbol": "PCM1",
  "term_label": "ciliary basal body"
}